{
  "gene_symbol": "ARL6IP4",
  "gene_name": "ADP-ribosylation factor-like protein 6-interacting protein 4",
  "term_label": "Unknown biological process",
  "term_id": "UNKNOWN:0002",
  "gene": "UniProtKB:Q66PJ3"
}